cellobiose transmembrane transporter activity [GO:0019191] (molecular function) Sources: GOC:mtg_transport, ISBN:0198506732, ISBN:0815340729 Relationships: is a type of disaccharide transmembrane transporter activity [GO:0015154]; is part of GO:0019533 Also known as: cellobiose permease activity Subtypes: protein-N(PI)-phosphohistidine-cellobiose phosphotransferase system transporter activity [GO:0022874] Definition: Enables the transfer of cellobiose from one side of a membrane to the other. Cellobiose, or 4-O-beta-D-glucopyranosyl-D-glucose, is a disaccharide that represents the basic repeating unit of cellulose.